regulation of phospholipid transport [GO:2001138] (biological process) Sources: GOC:obol Relationships: is a type of GO:0032368; regulates phospholipid transport [GO:0015914] Subtypes: regulation of phospholipid translocation [GO:0061091], regulation of phospholipid efflux [GO:1902994], negative regulation of phospholipid transport [GO:2001139], positive regulation of phospholipid transport [GO:2001140] Definition: Any process that modulates the frequency, rate or extent of phospholipid transport.